development of secondary sexual characteristics [GO:0045136] (biological process) Definition: The process whose specific outcome is the progression of the secondary sexual characteristics over time, from their formation to the mature structures. In humans, these include growth of axillary, chest, and pubic hair, voice changes, testicular/penile enlargement, breast development and menstrual periods. Development occurs in response to sex hormone secretion. Sources: GOC:ai Relationships: is a type of developmental process involved in reproduction [GO:0003006] Subtypes: development of secondary female sexual characteristics [GO:0046543], GO:0046544